establishment of protein localization to extracellular region [GO:0035592] (biological process) Also known as: establishment of protein localisation in extracellular region, establishment of protein localization in extracellular region Subtypes: GO:0009306, protein transport within extracellular region [GO:0071693] Relationships: is a type of GO:0045184 Sources: GOC:BHF, GOC:bf Definition: The directed movement of a protein to a specific location within the extracellular region.